isoleucine N-monooxygenase (oxime forming) activity [GO:0102001] (molecular function) Definition: Catalysis of the reaction: L-isoleucine + 2 O2 + 2 NADPH(4-) + 2 H+ = (E)-2-methylbutanal oxime + 2 NADP(3-) + carbon dioxide + 3 H2O. Relationships: is a type of oxidoreductase activity, acting on paired donors, with incorporation or reduction of molecular oxygen, NAD(P)H as one donor, and incorporation of one atom of oxygen [GO:0016709] Sources: EC:1.14.14.39